{
  "gene": "UniProtKB:Q60I27",
  "gene_symbol": "ALS2CL",
  "gene_name": "ALS2 C-terminal-like protein",
  "term_label": "small GTPase binding",
  "term_id": "GO:0031267"
}